{
  "gene_name": "Breast cancer metastasis-suppressor 1-like protein",
  "term_id": "GO:0070822",
  "gene": "UniProtKB:Q5PSV4",
  "term_label": "Sin3-type complex",
  "gene_symbol": "BRMS1L"
}